{
  "gene_symbol": "CPSF3",
  "gene": "UniProtKB:Q9UKF6",
  "term_label": "5'-3' RNA exonuclease activity",
  "term_id": "GO:0004534",
  "gene_name": "Cleavage and polyadenylation specificity factor subunit 3"
}